metanephric thick ascending limb development [GO:0072233] (biological process) Definition: The process whose specific outcome is the progression of the metanephric thick ascending limb over time, from its formation to the mature structure. The metanephric thick ascending limb is the last part of the metanephric loop of Henle. Its thick, mitochondria-rich epithelium characterizes the outer medulla, and is responsible for very avid active salt transport. At the macula densa, the thick ascending limb connects to the distal convoluted tubule. Sources: GOC:mtg_kidney_jan10 Also known as: metanephric TAL development Relationships: is a type of thick ascending limb development [GO:0072023]; is a type of metanephric nephron tubule development [GO:0072234]; is part of metanephric distal tubule development [GO:0072235]